{
  "term_label": "cytoskeleton organization",
  "term_id": "GO:0007010",
  "gene": "UniProtKB:Q9UKS6",
  "gene_name": "Protein kinase C and casein kinase substrate in neurons protein 3",
  "gene_symbol": "PACSIN3"
}